protocatechuate catabolic process, ortho-cleavage [GO:0019618] (biological process) Sources: MetaCyc:PROTOCATECHUATE-ORTHO-CLEAVAGE-PWY Definition: The chemical reactions and pathways resulting in the breakdown of protocatechuate, the anion of 3,4-dihydroxybenzoic acid, to yield beta-ketoadipate. Relationships: is a type of 3,4-dihydroxybenzoate catabolic process [GO:0019619]; is a type of GO:0043648; is a type of fatty acid derivative metabolic process [GO:1901568] Also known as: 3,4-dihydroxybenzoate catabolic process, ortho-cleavage, protocatechuate breakdown, ortho-cleavage, protocatechuate catabolic process to beta-ketoadipate, protocatechuate degradation, ortho-cleavage